L-histidine transmembrane transporter activity [GO:0005290] (molecular function) Also known as: L-histidine transporter activity, histidine/arginine/lysine/ornithine porter activity Relationships: is a type of aromatic amino acid transmembrane transporter activity [GO:0015173]; is a type of basic amino acid transmembrane transporter activity [GO:0015174]; is_a L-amino acid transmembrane transporter activity [GO:0015179]; is a type of azole transmembrane transporter activity [GO:1901474]; is part of L-histidine transmembrane transport [GO:0089709] Sources: GOC:ai, GOC:mtg_transport, ISBN:0815340729 Subtypes: GO:0005291, L-histidine:histamine antiporter activity [GO:0070907], L-histidine, sodium:proton antiporter activity [GO:0140832] Definition: Enables the transfer of L-histidine from one side of a membrane to the other. L-histidine is 2-amino-3-(1H-imidazol-4-yl)propanoic acid.